eyelid development in camera-type eye [GO:0061029] (biological process) Relationships: is a type of GO:0048856; is part of GO:0043010 Sources: GOC:dph, GOC:yaf Definition: The progression of the eyelid in a camera-type eye from its formation to the mature state. The eyelid is a membranous cover that helps protect and lubricate the eye.